{
  "term_label": "mitochondrial small ribosomal subunit",
  "gene": "UniProtKB:P82932",
  "gene_symbol": "MRPS6",
  "term_id": "GO:0005763",
  "gene_name": "Small ribosomal subunit protein bS6m"
}